{
  "gene": "UniProtKB:Q9BV36",
  "gene_symbol": "MLPH",
  "term_id": "UNKNOWN:0002",
  "gene_name": "Melanophilin",
  "term_label": "Unknown biological process"
}